{
  "gene_symbol": "H3-7",
  "gene_name": "Histone H3-7",
  "term_id": "GO:0031507",
  "term_label": "heterochromatin formation",
  "gene": "UniProtKB:Q5TEC6"
}